{
  "gene_name": "Serine_threonine-protein kinase TAO1",
  "term_id": "GO:0051493",
  "term_label": "regulation of cytoskeleton organization",
  "gene_symbol": "TAOK1",
  "gene": "UniProtKB:Q7L7X3"
}